establishment of vesicle localization [GO:0051650] (biological process) Also known as: establishment of vesicle localisation Relationships: is a type of vesicle localization [GO:0051648]; is a type of GO:0051649; is a type of establishment of organelle localization [GO:0051656] Subtypes: establishment of secretory granule localization [GO:0032254], vesicle targeting, cis-Golgi to rough endoplasmic reticulum [GO:0048206], synaptic vesicle transport [GO:0048489], establishment of pigment granule localization [GO:0051905], extracellular exosome macropinocytosis [GO:0061707], establishment of synaptic vesicle localization [GO:0097480], vesicle cytoskeletal trafficking [GO:0099518], dense core granule transport [GO:1901950], exosomal secretion [GO:1990182], dense core granule exocytosis [GO:1990504], clathrin-dependent extracellular exosome endocytosis [GO:1990771] Sources: GOC:ai Definition: The directed movement of a vesicle to a specific location.